{
  "gene_symbol": "ZFHX4",
  "gene": "UniProtKB:Q86UP3",
  "term_id": "GO:0005634",
  "gene_name": "Zinc finger homeobox protein 4",
  "term_label": "nucleus"
}